{
  "term_label": "intracellular calcium ion homeostasis",
  "gene_symbol": "STIM2",
  "gene": "UniProtKB:Q9P246",
  "gene_name": "Stromal interaction molecule 2",
  "term_id": "GO:0006874"
}